{
  "gene": "UniProtKB:Q9H2F9",
  "gene_symbol": "CCDC68",
  "term_id": "GO:0034454",
  "term_label": "microtubule anchoring at centrosome",
  "gene_name": "Coiled-coil domain-containing protein 68"
}